vitamin K metabolic process [GO:0042373] (biological process) Relationships: is a type of ketone metabolic process [GO:0042180] References: PMID:24489112 Sources: GOC:jl, https://en.wikipedia.org/wiki/Vitamin_K Subtypes: vitamin K biosynthetic process [GO:0042371], vitamin K catabolic process [GO:0042377] Also known as: naphthoquinone metabolic process, naphthoquinone metabolism, vitamin K metabolism Definition: The chemical reactions and pathways involving any of the forms of vitamin K, quinone-derived vitamins which are involved in the synthesis of blood-clotting factors in mammals. Vitamin K substances share a methylated naphthoquinone ring structure and vary in the aliphatic side chains attached to the molecule.